{
  "gene_symbol": "LSM7",
  "term_id": "GO:0071004",
  "gene_name": "U6 snRNA-associated Sm-like protein LSm7",
  "gene": "UniProtKB:Q9UK45",
  "term_label": "U2-type prespliceosome"
}